{
  "gene_symbol": "FMO3",
  "gene_name": "Flavin-containing monooxygenase 3",
  "gene": "UniProtKB:P31513",
  "term_label": "N,N-dimethylaniline monooxygenase activity",
  "term_id": "GO:0004499"
}